{
  "term_label": "interleukin-27 receptor binding",
  "gene_symbol": "IL27",
  "gene_name": "Interleukin-27 subunit alpha",
  "gene": "UniProtKB:Q8NEV9",
  "term_id": "GO:0045523"
}